{
  "term_id": "GO:0050772",
  "term_label": "positive regulation of axonogenesis",
  "gene_name": "Plexin-D1",
  "gene": "UniProtKB:Q9Y4D7",
  "gene_symbol": "PLXND1"
}